{
  "gene_symbol": "FHIP1A",
  "gene": "UniProtKB:Q05DH4",
  "gene_name": "FHF complex subunit HOOK-interacting protein 1A",
  "term_label": "Unknown molecular function",
  "term_id": "UNKNOWN:0001"
}